response to decalin [GO:1901493] (biological process) Definition: Any process that results in a change in state or activity of a cell or an organism (in terms of movement, secretion, enzyme production, gene expression, etc.) as a result of a decalin stimulus. Sources: GOC:TermGenie, GOC:mengo_curators Relationships: is_a GO:0042221